{
  "term_id": "GO:0006338",
  "gene": "UniProtKB:Q99873",
  "term_label": "chromatin remodeling",
  "gene_name": "Protein arginine N-methyltransferase 1",
  "gene_symbol": "PRMT1"
}